{
  "term_id": "UNKNOWN:0002",
  "gene_symbol": "HSF2BP",
  "term_label": "Unknown biological process",
  "gene_name": "Heat shock factor 2-binding protein",
  "gene": "UniProtKB:O75031"
}